cell wall macromolecule biosynthetic process [GO:0044038] (biological process) Also known as: cell wall macromolecule anabolism, cell wall macromolecule biosynthesis, cell wall macromolecule biosynthetic process at cellular level, cell wall macromolecule synthesis, cellular cell wall macromolecule biosynthetic process Subtypes: peptidoglycan biosynthetic process [GO:0009252], teichoic acid biosynthetic process [GO:0019350], cell wall glycoprotein biosynthetic process [GO:0031506], teichuronic acid biosynthetic process [GO:0050845], cell wall polysaccharide biosynthetic process [GO:0070592], mycolic acid biosynthetic process [GO:0071768] Relationships: is a type of GO:0009059; is a type of GO:0044036; is part of cell wall biogenesis [GO:0042546] Sources: GOC:go_curators Definition: The chemical reactions and pathways resulting in the formation of a macromolecule destined to form part of a cell wall.